{
  "gene": "UniProtKB:Q9UKV5",
  "term_id": "GO:0030968",
  "gene_symbol": "AMFR",
  "term_label": "endoplasmic reticulum unfolded protein response",
  "gene_name": "E3 ubiquitin-protein ligase AMFR"
}